{
  "term_id": "GO:0007155",
  "term_label": "cell adhesion",
  "gene": "UniProtKB:Q9HCB6",
  "gene_name": "Spondin-1",
  "gene_symbol": "SPON1"
}